postsynaptic actin cytoskeleton organization [GO:0098974] (BP) Definition: A process that is carried out at the cellular level which results in the assembly, arrangement of constituent parts, or disassembly of cytoskeletal structures comprising actin filaments and their associated proteins in the postsynaptic actin cytoskeleton. Sources: GOC:dos Relationships: is a type of GO:0030036; is a type of GO:0099188